{
  "term_id": "GO:0044183",
  "gene": "UniProtKB:O75190",
  "gene_name": "DnaJ homolog subfamily B member 6",
  "term_label": "protein folding chaperone",
  "gene_symbol": "DNAJB6"
}